{
  "term_id": "GO:0004394",
  "gene": "UniProtKB:Q7LGA3",
  "term_label": "heparan sulfate 2-sulfotransferase activity",
  "gene_name": "Heparan sulfate 2-O-sulfotransferase 1",
  "gene_symbol": "HS2ST1"
}